nicotinate-nucleotide adenylyltransferase activity [GO:0004515] (molecular function) Definition: Catalysis of the reaction: nicotinate beta-D-ribonucleotide + ATP + H+ = deamido-NAD+ + diphosphate. Sources: RHEA:22860 Also known as: ATP:nicotinate-nucleotide adenylyltransferase activity, nicotinic acid mononucleotide adenylyltransferase, ATP:nicotinate-ribonucleotide adenylyltransferase activity, NaMN-ATase activity, deamido-NAD(+) diphosphorylase activity, deamido-NAD(+) pyrophosphorylase activity, deamido-NAD+ pyrophosphorylase activity, deamidonicotinamide adenine dinucleotide pyrophosphorylase activity, nicotinate mononucleotide adenylyltransferase activity Relationships: is_a adenylyltransferase activity [GO:0070566]